{
  "gene_name": "Zinc finger and BTB domain-containing protein 32",
  "term_id": "GO:0001817",
  "gene_symbol": "ZBTB32",
  "term_label": "regulation of cytokine production",
  "gene": "UniProtKB:Q9Y2Y4"
}